{
  "gene_name": "Anaphase-promoting complex subunit CDC26",
  "gene_symbol": "CDC26",
  "term_id": "GO:0005680",
  "gene": "UniProtKB:Q8NHZ8",
  "term_label": "anaphase-promoting complex"
}